{
  "gene_symbol": "INPP5F",
  "term_label": "phosphatidylinositol-4-phosphate phosphatase activity",
  "gene_name": "Phosphatidylinositide phosphatase SAC2",
  "term_id": "GO:0043812",
  "gene": "UniProtKB:Q9Y2H2"
}